{
  "gene_name": "Diacylglycerol kinase delta",
  "term_id": "GO:0006654",
  "gene": "UniProtKB:Q16760",
  "gene_symbol": "DGKD",
  "term_label": "phosphatidic acid biosynthetic process"
}